{
  "term_id": "GO:0005634",
  "gene_symbol": "DMRTA2",
  "gene": "UniProtKB:Q96SC8",
  "gene_name": "Doublesex- and mab-3-related transcription factor A2",
  "term_label": "nucleus"
}